{
  "gene_name": "PRAME family member 7",
  "gene_symbol": "PRAMEF7",
  "term_label": "proteasome-mediated ubiquitin-dependent protein catabolic process",
  "term_id": "GO:0043161",
  "gene": "UniProtKB:Q5VXH5"
}